cholesterol transfer activity [GO:0120020] (molecular function) Also known as: cholesterol transporter activity, cholesterol carrier activity, intermembrane cholesterol transfer activity Definition: Removes cholesterol from a membrane or a monolayer lipid particle, transports it through the aqueous phase while protected in a hydrophobic pocket, and brings it to an acceptor membrane or lipid particle. Subtypes: phosphatidylinositol-4-phosphate-cholesterol exchange activity [GO:0160291] References: PMID:20823909, PMID:24220498, PMID:25797198 Sources: GOC:krc Relationships: is_a sterol transfer activity [GO:0120015]; has part GO:0015485